{
  "gene": "UniProtKB:Q9Y3D8",
  "gene_symbol": "AK6",
  "term_label": "cytoplasm",
  "gene_name": "Adenylate kinase isoenzyme 6",
  "term_id": "GO:0005737"
}